{
  "gene": "UniProtKB:Q9H0R8",
  "gene_name": "Gamma-aminobutyric acid receptor-associated protein-like 1",
  "gene_symbol": "GABARAPL1",
  "term_id": "GO:0008429",
  "term_label": "phosphatidylethanolamine binding"
}